melanosome assembly [GO:1903232] (biological process) Relationships: is a type of melanosome organization [GO:0032438]; is_a organelle assembly [GO:0070925] Definition: The aggregation, arrangement and bonding together of a set of components to form a melanosome, a tissue-specific, membrane-bounded cytoplasmic organelle within which melanin pigments are synthesized and stored. References: PMID:22511774 Sources: GOC:PARL, GOC:TermGenie, GOC:bf, GO_REF:0000079 Also known as: melanosome formation